ABC-type indole transporter activity [GO:0160080] (molecular function) Relationships: is_a GO:0140359 Definition: Enables the transfer of a solute or solutes from one side of a membrane to the other according to the reaction: ATP + H2O + indole(in) = ADP + phosphate + indole(out). References: PMID:37146609